{
  "term_id": "UNKNOWN:0001",
  "term_label": "Unknown molecular function",
  "gene": "UniProtKB:P51572",
  "gene_name": "B-cell receptor-associated protein 31",
  "gene_symbol": "BCAP31"
}